RNA polymerase binding [GO:0070063] (molecular function) Definition: Binding to an RNA polymerase molecule or complex. Sources: GOC:BHF, GOC:mah, GOC:txnOH Relationships: is a type of enzyme binding [GO:0019899] Subtypes: GO:0001050, RNA polymerase core enzyme binding [GO:0043175]